{
  "term_id": "GO:0016485",
  "gene_name": "Carboxypeptidase N catalytic chain",
  "gene_symbol": "CPN1",
  "term_label": "protein processing",
  "gene": "UniProtKB:P15169"
}